levanase activity [GO:0031219] (molecular function) Also known as: levan hydrolase activity, 2,6-beta-D-fructan fructanohydrolase activity Definition: Catalysis of the random hydrolysis of 2,6-beta-D-fructofuranosidic linkages in 2,6-beta-D-fructans (levans) containing more than 3 fructose units. Sources: EC:3.2.1.65, GOC:mlg Relationships: is a type of hydrolase activity, hydrolyzing O-glycosyl compounds [GO:0004553]